{
  "gene": "UniProtKB:Q13309",
  "gene_name": "S-phase kinase-associated protein 2",
  "term_id": "GO:1990756",
  "gene_symbol": "SKP2",
  "term_label": "ubiquitin-like ligase-substrate adaptor activity"
}